{
  "term_label": "sequence-specific double-stranded DNA binding",
  "gene_name": "Homeobox protein unc-4 homolog",
  "gene_symbol": "UNCX",
  "gene": "UniProtKB:A6NJT0",
  "term_id": "GO:1990837"
}